{
  "gene_symbol": "IGLV3-19",
  "term_label": "Unknown molecular function",
  "gene_name": "Immunoglobulin lambda variable 3-19",
  "gene": "UniProtKB:P01714",
  "term_id": "UNKNOWN:0001"
}